{
  "term_id": "UNKNOWN:0002",
  "gene": "UniProtKB:P11182",
  "gene_symbol": "DBT",
  "term_label": "Unknown biological process",
  "gene_name": "Lipoamide acyltransferase component of branched-chain alpha-keto acid dehydrogenase complex, mitochondrial"
}